{
  "term_id": "UNKNOWN:0002",
  "gene": "UniProtKB:Q8NGG0",
  "term_label": "Unknown biological process",
  "gene_symbol": "OR8J3",
  "gene_name": "Olfactory receptor 8J3"
}